{
  "term_label": "Unknown biological process",
  "gene_name": "SAFB-like transcription modulator",
  "gene": "UniProtKB:Q9NWH9",
  "term_id": "UNKNOWN:0002",
  "gene_symbol": "SLTM"
}